acetylcholine receptor activity [GO:0015464] (molecular function) Regulation: regulated by acetylcholine receptor regulator activity [GO:0030548]; RO_0002213 by acetylcholine receptor activator activity [GO:0030549]; negatively regulated by GO:0030550 Sources: GOC:jl, GOC:signaling Relationships: is a type of transmembrane signaling receptor activity [GO:0004888]; is a type of postsynaptic neurotransmitter receptor activity [GO:0098960]; BFO_0000050 synaptic transmission, cholinergic [GO:0007271]; has part acetylcholine binding [GO:0042166] Definition: Combining with an acetylcholine receptor ligand and transmitting the signal from one side of the membrane to the other to initiate a change in cell activity. Subtypes: G protein-coupled acetylcholine receptor activity [GO:0016907] Note: For nicotinic acetylcholine receptors that act as ion channels, instead use 'acetylcholine-gated cation channel activity ; GO:0022848'.